{
  "term_label": "protein phosphatase activator activity",
  "term_id": "GO:0072542",
  "gene_name": "Serine_threonine-protein phosphatase 2A 56 kDa regulatory subunit beta isoform",
  "gene": "UniProtKB:Q15173",
  "gene_symbol": "PPP2R5B"
}